response to phosphatidylethanolamine [GO:1905711] (biological process) Subtypes: cellular response to phosphatidylethanolamine [GO:1905712] Also known as: response to PE, response to PtdEtn, response to phosphatidyl(amino)ethanols, response to phosphatidylethanolamines Relationships: is a type of response to lipid [GO:0033993]; is a type of response to organophosphorus [GO:0046683]; is a type of response to oxygen-containing compound [GO:1901700] References: PMID:1657995 Sources: GOC:TermGenie, GO_REF:0000071 Definition: Any process that results in a change in state or activity of a cell or an organism (in terms of movement, secretion, enzyme production, gene expression, etc.) as a result of a phosphatidylethanolamine stimulus.